{
  "gene_symbol": "GET4",
  "gene": "UniProtKB:Q7L5D6",
  "term_id": "GO:0005829",
  "gene_name": "Golgi to ER traffic protein 4 homolog",
  "term_label": "cytosol"
}